{
  "gene_symbol": "KLF16",
  "gene_name": "Krueppel-like factor 16",
  "term_id": "GO:0006357",
  "term_label": "regulation of transcription by RNA polymerase II",
  "gene": "UniProtKB:Q9BXK1"
}